neural crest cell migration involved in heart formation [GO:0003147] (BP) Relationships: is a type of neural crest cell migration [GO:0001755]; is a type of cell migration involved in heart formation [GO:0060974]; is part of GO:0061308 Sources: GOC:mtg_heart Definition: The characteristic movement of a cell from the dorsal ridge of the neural tube towards the heart and that contributes to heart formation.